{
  "term_id": "GO:0003009",
  "gene": "UniProtKB:P02585",
  "gene_symbol": "TNNC2",
  "gene_name": "Troponin C, skeletal muscle",
  "term_label": "skeletal muscle contraction"
}